{
  "gene": "UniProtKB:Q9UBL0",
  "term_label": "Unknown biological process",
  "gene_name": "cAMP-regulated phosphoprotein 21",
  "gene_symbol": "ARPP21",
  "term_id": "UNKNOWN:0002"
}